{
  "term_id": "UNKNOWN:0002",
  "gene": "UniProtKB:Q6ZW13",
  "gene_symbol": "C16orf86",
  "term_label": "Unknown biological process",
  "gene_name": "Uncharacterized protein C16orf86"
}